{
  "term_id": "GO:0086091",
  "term_label": "regulation of heart rate by cardiac conduction",
  "gene": "UniProtKB:Q9UJ90",
  "gene_symbol": "KCNE5",
  "gene_name": "Potassium voltage-gated channel subfamily E regulatory beta subunit 5"
}